telomeric DNA binding [GO:0042162] (molecular function) Sources: GOC:jl, SO:0000624 Relationships: is a type of GO:0043565 Subtypes: GO:0003691, single-stranded telomeric DNA binding [GO:0043047], telomeric G-quadruplex DNA binding [GO:0061849], double-stranded/single-stranded junction telomeric DNA binding [GO:0090655] Also known as: telomere binding, telomeric repeat binding Definition: Binding to a telomere, a specific structure at the end of a linear chromosome required for the integrity and maintenance of the end.